{
  "gene": "UniProtKB:O76041",
  "term_label": "Z disc",
  "term_id": "GO:0030018",
  "gene_name": "Nebulette",
  "gene_symbol": "NEBL"
}